{
  "term_id": "GO:0004842",
  "term_label": "ubiquitin-protein transferase activity",
  "gene_name": "E3 ubiquitin-protein ligase TRIM36",
  "gene_symbol": "TRIM36",
  "gene": "UniProtKB:Q9NQ86"
}